{
  "gene_name": "Ubiquitin-conjugating enzyme E2 Z",
  "gene": "UniProtKB:Q9H832",
  "term_label": "negative regulation of apoptotic process",
  "term_id": "GO:0043066",
  "gene_symbol": "UBE2Z"
}